{
  "term_label": "uridine kinase activity",
  "gene_name": "Uridine-cytidine kinase 1",
  "term_id": "GO:0004849",
  "gene": "UniProtKB:Q9HA47",
  "gene_symbol": "UCK1"
}